positive regulation of odontogenesis [GO:0042482] (biological process) Sources: GOC:jl Also known as: positive regulation of tooth development, up regulation of odontogenesis, up-regulation of odontogenesis, upregulation of odontogenesis, activation of odontogenesis, positive regulation of odontogenesis of calcareous or chitinous tooth, stimulation of odontogenesis Relationships: is a type of regulation of odontogenesis [GO:0042481]; is a type of positive regulation of animal organ morphogenesis [GO:0110110]; positively regulates odontogenesis [GO:0042476] Subtypes: positive regulation of odontogenesis of dentin-containing tooth [GO:0042488] Definition: Any process that activates or increases the frequency, rate or extent of the formation and development of a tooth or teeth.